ethanol metabolic process [GO:0006067] (biological process) Also known as: ethanol metabolism Definition: The chemical reactions and pathways involving ethanol, CH3-CH2-OH, a colorless, water-miscible, flammable liquid produced by alcoholic fermentation. Relationships: is a type of GO:0034308 Sources: GOC:ai, ISBN:0198506732 Subtypes: ethanol catabolic process [GO:0006068], GO:0006115, acetyl-CoA biosynthetic process from ethanol [GO:0019431], pyruvate fermentation to ethanol [GO:0019655], glucose catabolic process to D-lactate and ethanol [GO:0019656], GO:0019664, D-xylose catabolic process to ethanol [GO:0044577]